positive regulation of L-lysine import across plasma membrane [GO:1905010] (biological process) Also known as: positive regulation of L-lysine import into cell, up regulation of L-lysine import into cell, up-regulation of L-lysine import into cell, upregulation of L-lysine import into cell, activation of L-lysine import into cell Definition: Any process that activates or increases the frequency, rate or extent of L-lysine import into cell. Relationships: is a type of positive regulation of organic acid transport [GO:0032892]; is a type of positive regulation of transmembrane transport [GO:0034764]; is a type of GO:0051957; is a type of regulation of L-lysine import across plasma membrane [GO:1905008]; positively regulates L-lysine import across plasma membrane [GO:0097639] References: PMID:7499219 Sources: GOC:TermGenie, GO_REF:0000058